dTTP biosynthetic process [GO:0006235] (BP) Also known as: dTTP anabolism, dTTP biosynthesis, dTTP formation, dTTP synthesis Sources: ISBN:0198506732 Definition: The chemical reactions and pathways resulting in the formation of dTTP, deoxyribosylthymine triphosphate. Relationships: is a type of pyrimidine deoxyribonucleoside triphosphate biosynthetic process [GO:0009212]; is a type of pyrimidine deoxyribonucleotide biosynthetic process [GO:0009221]; is a type of GO:0046075